{
  "term_id": "GO:2000344",
  "term_label": "positive regulation of acrosome reaction",
  "gene_name": "Probable inactive serine protease 37",
  "gene": "UniProtKB:A4D1T9",
  "gene_symbol": "PRSS37"
}